chaperone-mediated autophagy translocation complex assembly [GO:1904763] (biological process) References: PMID:18644871 Sources: GOC:PARL, GOC:TermGenie, GOC:pad, GO_REF:0000079 Relationships: is_a protein-containing complex assembly [GO:0065003]; BFO_0000050 chaperone-mediated autophagy [GO:0061684] Also known as: CMA translocation complex assembly, CMA translocation complex formation, chaperone-mediated autophagy translocation complex formation, CMA receptor complex assembly, CMA receptor complex formation, chaperone-mediated autophagy receptor complex assembly, chaperone-mediated autophagy receptor complex formation Definition: The aggregation, arrangement and bonding together of a set of components to form a chaperone-mediated autophagy translocation complex.